voltage-gated calcium channel activity involved in positive regulation of presynaptic cytosolic calcium levels [GO:0099635] (molecular function) Definition: Positive regulation of presynaptic cytosolic calcium ion concentrations via the directed movement of calcium ions across the plasma-membrane into the cytosol via the action of voltage-gated calcium ion channels. This is the first step in synaptic transmission. Sources: GOC:dos Relationships: is a type of GO:0005245; is part of induction of synaptic vesicle exocytosis by positive regulation of presynaptic cytosolic calcium ion concentration [GO:0099703]; BFO_0000066 presynapse [GO:0098793]